{
  "gene_symbol": "CAAP1",
  "gene_name": "Caspase activity and apoptosis inhibitor 1",
  "gene": "UniProtKB:Q9H8G2",
  "term_label": "Unknown biological process",
  "term_id": "UNKNOWN:0002"
}